 [IAO:0000231]